{
  "term_id": "UNKNOWN:0002",
  "gene_name": "Keratin-associated protein 4-6",
  "gene": "UniProtKB:Q9BYQ5",
  "term_label": "Unknown biological process",
  "gene_symbol": "KRTAP4-6"
}